{
  "term_label": "bicellular tight junction",
  "gene_symbol": "CLDN22",
  "gene": "UniProtKB:Q8N7P3",
  "gene_name": "Claudin-22",
  "term_id": "GO:0005923"
}